{
  "gene_symbol": "DUSP8",
  "gene_name": "Dual specificity protein phosphatase 8",
  "gene": "UniProtKB:Q13202",
  "term_label": "cytoplasm",
  "term_id": "GO:0005737"
}